{
  "gene_symbol": "KRT83",
  "term_id": "GO:0030280",
  "gene": "UniProtKB:P78385",
  "term_label": "structural constituent of skin epidermis",
  "gene_name": "Keratin, type II cuticular Hb3"
}